{
  "term_label": "C-C chemokine binding",
  "gene_name": "C-X-C chemokine receptor type 4",
  "gene_symbol": "CXCR4",
  "gene": "UniProtKB:P61073",
  "term_id": "GO:0019957"
}